{
  "gene_name": "Uncharacterized protein",
  "term_id": "UNKNOWN:0001",
  "gene_symbol": "A0A0G2JLW4",
  "term_label": "Unknown molecular function",
  "gene": "UniProtKB:A0A0G2JLW4"
}